glandular epithelial cell differentiation [GO:0002067] (biological process) Subtypes: thyroid-stimulating hormone-secreting cell differentiation [GO:0060129], secretory columnal luminar epithelial cell differentiation involved in prostate glandular acinus development [GO:0060528], squamous basal epithelial stem cell differentiation involved in prostate gland acinus development [GO:0060529], adrenal chromaffin cell differentiation [GO:0061104], acinar cell differentiation [GO:0090425] Relationships: is a type of GO:0002065 Definition: The process in which a relatively unspecialized cell acquires specialized features of a glandular epithelial cell. A glandular epithelial cell is a columnar/cuboidal epithelial cell found in a two dimensional sheet with a free surface exposed to the lumen of a gland. Sources: GOC:dph